{
  "term_label": "intermediate filament bundle assembly",
  "gene_name": "Plakophilin-2",
  "gene_symbol": "PKP2",
  "gene": "UniProtKB:Q99959",
  "term_id": "GO:0045110"
}